{
  "gene_symbol": "BCL2L10",
  "term_id": "GO:0005741",
  "gene_name": "Bcl-2-like protein 10",
  "gene": "UniProtKB:Q9HD36",
  "term_label": "mitochondrial outer membrane"
}